cellular response to zinc ion [GO:0071294] (biological process) Definition: Any process that results in a change in state or activity of a cell (in terms of movement, secretion, enzyme production, gene expression, etc.) as a result of a zinc ion stimulus. Also known as: cellular response to zinc Relationships: is a type of response to zinc ion [GO:0010043]; is a type of GO:0071248 Sources: GOC:mah